type 1 neuropeptide Y receptor binding [GO:0031842] (molecular function) Also known as: type 1 neuropeptide Y receptor ligand Sources: GOC:mah, GOC:nln Relationships: is a type of neuropeptide Y receptor binding [GO:0031841] Definition: Binding to a type 1 neuropeptide Y receptor.